{
  "gene": "UniProtKB:Q9GZM5",
  "gene_name": "Protein YIPF3",
  "gene_symbol": "YIPF3",
  "term_id": "UNKNOWN:0002",
  "term_label": "Unknown biological process"
}